{
  "gene_name": "cAMP-specific 3',5'-cyclic phosphodiesterase 7B",
  "gene_symbol": "PDE7B",
  "term_label": "negative regulation of cAMP/PKA signal transduction",
  "term_id": "GO:0141162",
  "gene": "UniProtKB:Q9NP56"
}